{
  "gene": "UniProtKB:Q96RE9",
  "term_label": "nucleus",
  "gene_name": "Zinc finger protein 300",
  "term_id": "GO:0005634",
  "gene_symbol": "ZNF300"
}